eosinophil degranulation [GO:0043308] (biological process) Regulation: regulated by regulation of eosinophil degranulation [GO:0043309]; negatively regulated by negative regulation of eosinophil degranulation [GO:0043310]; positively regulated by GO:0043311 Also known as: eosinophil granule exocytosis Relationships: is a type of leukocyte degranulation [GO:0043299]; is part of GO:0002278; is part of eosinophil mediated immunity [GO:0002447] Definition: The regulated exocytosis of secretory granules containing preformed mediators such as major basic protein, eosinophil peroxidase, and eosinophil cationic protein by an eosinophil. Sources: ISBN:0781735149